myoblast fate determination involved in skeletal muscle regeneration [GO:0014837] (biological process) Definition: The process in which a satellite cell becomes capable of differentiating autonomously into a myoblast regardless of its environment; upon determination, the cell fate cannot be reversed. This occurs as part of skeletal muscle regeneration. A myoblast is a mononucleate cell type that, by fusion with other myoblasts, gives rise to the myotubes that eventually develop into skeletal muscle fibers. Relationships: is a type of myoblast fate determination [GO:0007518]; is part of GO:0014836 References: PMID:16607119 Sources: CL:0000056, GOC:ef, GOC:mtg_muscle